{
  "term_label": "extrinsic apoptotic signaling pathway via death domain receptors",
  "term_id": "GO:0008625",
  "gene_symbol": "TNF",
  "gene_name": "Tumor necrosis factor",
  "gene": "UniProtKB:P01375"
}